{
  "term_label": "cell migration",
  "gene_name": "Syndecan-4",
  "gene": "UniProtKB:P31431",
  "gene_symbol": "SDC4",
  "term_id": "GO:0016477"
}